{
  "term_label": "nucleus",
  "term_id": "GO:0005634",
  "gene_symbol": "BAG4",
  "gene_name": "BAG family molecular chaperone regulator 4",
  "gene": "UniProtKB:O95429"
}